{
  "gene_name": "Small lysine-rich protein 1",
  "gene_symbol": "SMKR1",
  "term_label": "Unknown molecular function",
  "term_id": "UNKNOWN:0001",
  "gene": "UniProtKB:H3BMG3"
}